{
  "gene_name": "tRNA-splicing endonuclease subunit Sen54",
  "gene_symbol": "TSEN54",
  "gene": "UniProtKB:Q7Z6J9",
  "term_id": "UNKNOWN:0001",
  "term_label": "Unknown molecular function"
}